{
  "gene_symbol": "HIF1A",
  "term_label": "DNA-binding transcription factor activity, RNA polymerase II-specific",
  "gene": "UniProtKB:Q16665",
  "gene_name": "Hypoxia-inducible factor 1-alpha",
  "term_id": "GO:0000981"
}